queuosine transmembrane transporter activity [GO:0160286] (molecular function) Definition: Enables the transfer of queuosine from one side of a membrane to the other according to the reaction: queuosine(out) = queuosine(in). Relationships: is a type of nucleoside transmembrane transporter activity [GO:0005337]; is part of queuosine import across plasma membrane [GO:0160287] References: PMID:40526720